{
  "term_label": "calcium ion transmembrane transporter activity",
  "gene_symbol": "TMEM165",
  "term_id": "GO:0015085",
  "gene_name": "Transmembrane protein 165",
  "gene": "UniProtKB:Q9HC07"
}